{
  "gene_name": "VIP peptides",
  "gene": "UniProtKB:P01282",
  "term_id": "GO:0141163",
  "term_label": "positive regulation of cAMP/PKA signal transduction",
  "gene_symbol": "VIP"
}